{
  "term_id": "GO:0006376",
  "term_label": "mRNA splice site recognition",
  "gene": "UniProtKB:Q92879",
  "gene_symbol": "CELF1",
  "gene_name": "CUGBP Elav-like family member 1"
}